piRNA-mediated heterochromatin formation [GO:0140966] (biological process) References: PMID:23329111 Definition: The formation of heterochromatin into a heterochromatin domain, enriched in histone H3 methylated on lysine 9 (H3K9me), by a process mediated by a Piwi-associated RNA (piRNA). Relationships: is_a regulatory ncRNA-mediated heterochromatin formation [GO:0031048] Subtypes: transposable element silencing by piRNA-mediated heterochromatin formation [GO:0141006], gene silencing by piRNA-directed DNA methylation [GO:0141176] Also known as: piRNA-directed heterochromatin formation, piwiRNA-directed heterochromatin formation